regulation of eIF2 alpha phosphorylation by dsRNA [GO:0060735] (biological process) Definition: Any process that modulates the rate, frequency, or extent of eIF2 alpha phosphorylation as a cellular response to double-stranded RNA. Sources: GOC:dph, GOC:tb Also known as: regulation of eIF2 alpha phosphorylation by double-stranded RNA, regulation of eIF2 alpha phosphorylation by PKR Relationships: is a type of regulation of protein phosphorylation [GO:0001932]; is a type of GO:0006446; is a type of regulation of cellular response to stress [GO:0080135]; is part of cellular response to dsRNA [GO:0071359]; regulates GO:0010998